{
  "gene": "UniProtKB:P60368",
  "term_id": "UNKNOWN:0003",
  "gene_name": "Keratin-associated protein 10-2",
  "gene_symbol": "KRTAP10-2",
  "term_label": "Unknown cellular component"
}